{
  "term_id": "GO:0070098",
  "term_label": "chemokine-mediated signaling pathway",
  "gene_symbol": "CXCL10",
  "gene_name": "C-X-C motif chemokine 10",
  "gene": "UniProtKB:P02778"
}